L-threonine import across plasma membrane [GO:1903807] (biological process) Definition: The directed movement of L-threonine from outside of a cell, across the plasma membrane and into the cytosol. References: PMID:23895341 Sources: GOC:TermGenie, GO_REF:0000075 Relationships: is a type of organic cation transport [GO:0015695]; is a type of GO:0015826; is a type of amino acid import across plasma membrane [GO:0089718]; is a type of GO:1902475 Also known as: L-threonine import, L-threonine import into cell, L-threonine uptake Regulation: regulated by regulation of L-threonine import across plasma membrane [GO:1900926]; negatively regulated by negative regulation of L-threonine import across plasma membrane [GO:1900927]; positively regulated by positive regulation of L-threonine import across plasma membrane [GO:1900928]